maltose transport [GO:0015768] (biological process) Definition: The directed movement of maltose into, out of or within a cell, or between cells, by means of some agent such as a transporter or pore. Maltose is the disaccharide 4-O-alpha-D-glucopyranosyl-D-glucopyranose, an intermediate in the catabolism of glycogen and starch. Sources: GOC:ai Relationships: is a type of disaccharide transport [GO:0015766] Subtypes: maltose transmembrane transport [GO:1904981] Regulation: regulated by regulation of maltose transport [GO:1902343]; negatively regulated by GO:1902344; RO_0002213 by positive regulation of maltose transport [GO:1902345]